{
  "gene_name": "Cytochrome P450 1A2",
  "gene_symbol": "CYP1A2",
  "term_id": "GO:0006706",
  "gene": "UniProtKB:P05177",
  "term_label": "steroid catabolic process"
}